{
  "gene_name": "Calsyntenin-2",
  "gene": "UniProtKB:Q9H4D0",
  "gene_symbol": "CLSTN2",
  "term_id": "GO:0098839",
  "term_label": "postsynaptic density membrane"
}